{
  "term_id": "GO:0140682",
  "gene_symbol": "KDM1A",
  "gene_name": "Lysine-specific histone demethylase 1A",
  "term_label": "FAD-dependent H3K4me/H3K4me3 demethylase activity",
  "gene": "UniProtKB:O60341"
}